{
  "gene": "UniProtKB:O95996",
  "term_id": "GO:0007399",
  "gene_name": "Adenomatous polyposis coli protein 2",
  "term_label": "nervous system development",
  "gene_symbol": "APC2"
}